hormone-mediated signaling pathway [GO:0009755] (biological process) Definition: The series of molecular signals mediated by the detection of a hormone. Sources: GOC:sm Also known as: hormone mediated signalling Relationships: is a type of GO:0007165; is part of GO:0032870 Subtypes: thyroid hormone receptor signaling pathway [GO:0002154], GO:0008628, auxin-activated signaling pathway [GO:0009734], cytokinin-activated signaling pathway [GO:0009736], abscisic acid-activated signaling pathway [GO:0009738], GO:0009867, ethylene-activated signaling pathway [GO:0009873], gibberellin mediated signaling pathway [GO:0010476], adiponectin-activated signaling pathway [GO:0033211], juvenile hormone mediated signaling pathway [GO:0035626], prolactin signaling pathway [GO:0038161], somatostatin signaling pathway [GO:0038170], steroid hormone receptor signaling pathway [GO:0043401], retinoic acid receptor signaling pathway [GO:0048384], vitamin D receptor signaling pathway [GO:0070561]